prostatic bud formation [GO:0060513] (biological process) Definition: The morphogenetic process in which a region of the fetal urogenital sinus epithelium is specified to become the prostate, resulting in prostate bud outgrowth. Regulation: regulated by regulation of prostatic bud formation [GO:0060685]; negatively regulated by GO:0060686 Relationships: is a type of GO:0016331; is_a animal organ formation [GO:0048645]; is a type of morphogenesis of an epithelial bud [GO:0060572]; is a type of lateral sprouting from an epithelium [GO:0060601]; is a type of GO:0060740 References: PMID:18977204 Sources: GOC:dph Also known as: primary prostate bud formation, prostate ductal budding, prostate gland formation